{
  "term_id": "UNKNOWN:0002",
  "term_label": "Unknown biological process",
  "gene": "UniProtKB:Q8NGF6",
  "gene_name": "Olfactory receptor 10W1",
  "gene_symbol": "OR10W1"
}